{
  "term_label": "Unknown cellular component",
  "gene": "UniProtKB:Q05513",
  "term_id": "UNKNOWN:0003",
  "gene_symbol": "PRKCZ",
  "gene_name": "Protein kinase C zeta type"
}